{
  "gene": "UniProtKB:Q9NZ32",
  "term_id": "GO:0005200",
  "gene_name": "Actin-related protein 10",
  "gene_symbol": "ACTR10",
  "term_label": "structural constituent of cytoskeleton"
}